flagella connector [GO:0120118] (cellular component) Relationships: is a type of GO:0030054 Note: Note that we deem cilium and microtubule-based flagellum to be equivalent; the primary term name reflects frequency of use. Definition: A mobile transmembrane junction at the tip of the flagellum of some kinetoplastid species linking the tip of a new growing flagellum to an older flagellum. References: PMID:11641501, PMID:15075226, PMID:16954145, PMID:26820516